{
  "gene_name": "Solute carrier family 22 member 10",
  "gene": "UniProtKB:Q63ZE4",
  "term_id": "UNKNOWN:0001",
  "term_label": "Unknown molecular function",
  "gene_symbol": "SLC22A10"
}